tellurite methyltransferase activity [GO:0035797] (molecular function) References: PMID:11053398, PMID:21244361 Sources: GOC:bf, GOC:kad Definition: Catalysis of the transfer of a methyl group from S-adenosyl-L-methionine to tellurite [TeO3(2-)]. Methylated derivatives of tellurite include Te(CH3)2 (dimethyltelluride) and Te2(CH3)2 (dimethylditelluride). Also known as: tellurite methylase activity, S-adenosyl-L-methionine-dependent tellurite methyltransferase activity, SAM-dependent tellurite methyltransferase activity Relationships: is a type of S-adenosylmethionine-dependent methyltransferase activity [GO:0008757]